viral translation [GO:0019081] (biological process) Also known as: viral protein anabolism, viral protein biosynthesis, viral protein biosynthetic process, viral protein formation, viral protein synthesis Definition: A process by which viral mRNA is translated into viral protein, using the host cellular machinery. Regulation: regulated by regulation of viral translation [GO:1904971]; negatively regulated by negative regulation of viral translation [GO:1904972]; positively regulated by positive regulation of viral translation [GO:1904973] Sources: GOC:bf, GOC:jl, ISBN:0781702534 Subtypes: viral translational shunt [GO:0039704] Relationships: is a type of viral process [GO:0016032]; is part of viral gene expression [GO:0019080]